{
  "gene_name": "Collagen alpha-1(XV) chain",
  "term_id": "GO:0030020",
  "gene": "UniProtKB:P39059",
  "term_label": "extracellular matrix structural constituent conferring tensile strength",
  "gene_symbol": "COL15A1"
}